paraxial mesoderm morphogenesis [GO:0048340] (BP) Relationships: is a type of GO:0048332; is a type of mesenchyme morphogenesis [GO:0072132]; is part of GO:0048339 Definition: The process in which the anatomical structures of the paraxial mesoderm are generated and organized. Sources: GOC:go_curators